{
  "gene_symbol": "RAB27B",
  "gene": "UniProtKB:O00194",
  "term_id": "GO:0016324",
  "term_label": "apical plasma membrane",
  "gene_name": "Ras-related protein Rab-27B"
}